inositol-1,3,4,6-tetrakisphosphate 1-phosphatase activity [GO:0052831] (molecular function) Definition: Catalysis of the reaction: inositol-1,3,4,6-tetrakisphosphate + H2O = inositol-3,4,6-trisphosphate + phosphate. Sources: GOC:ai Relationships: is a type of inositol tetrakisphosphate phosphatase activity [GO:0052743]